{
  "gene": "UniProtKB:P01571",
  "gene_symbol": "IFNA17",
  "term_id": "GO:0002323",
  "term_label": "natural killer cell activation involved in immune response",
  "gene_name": "Interferon alpha-17"
}